{
  "gene": "UniProtKB:P27635",
  "term_id": "GO:0022625",
  "gene_symbol": "RPL10",
  "term_label": "cytosolic large ribosomal subunit",
  "gene_name": "Large ribosomal subunit protein uL16"
}